{
  "term_label": "clathrin adaptor activity",
  "gene_symbol": "STON2",
  "term_id": "GO:0035615",
  "gene": "UniProtKB:Q8WXE9",
  "gene_name": "Stonin-2"
}